{
  "term_label": "Unknown cellular component",
  "gene": "UniProtKB:A1L429",
  "gene_symbol": "GAGE12E",
  "gene_name": "G antigen 12B_C_D_E",
  "term_id": "UNKNOWN:0003"
}